dendritic branch [GO:0044307] (cellular component) Also known as: dendrite branch, secondary dendrite Relationships: is a type of GO:0030425 Sources: GOC:aruk, GOC:bc, NIF_Subcellular:sao884265541 Definition: A dendrite arising from another dendrite.